platelet rolling [GO:0160015] (biological process) Relationships: is a type of GO:0034113 References: PMID:29018081 Sources: GOC:sl Regulation: regulated by regulation of platelet rolling [GO:0160017]; positively regulated by positive regulation of platelet rolling [GO:0160018]; negatively regulated by negative regulation of platelet rolling [GO:0160019] Definition: Transient adhesive interactions between platelets and endothelial cells lining blood vessels. Carbohydrates on circulating platelets bind selectins or other molecules on the vessel wall causing the platelets to slow down and roll along the inner surface of the vessel wall. During this rolling motion, transitory bonds are formed and broken between surface molecules of platelets and endothelium.